{
  "gene_name": "Inactive tyrosine-protein kinase 7",
  "gene_symbol": "PTK7",
  "term_id": "GO:0050808",
  "gene": "UniProtKB:Q13308",
  "term_label": "synapse organization"
}